{
  "gene_name": "Histone acetyltransferase KAT7",
  "term_id": "GO:0000785",
  "gene_symbol": "KAT7",
  "gene": "UniProtKB:O95251",
  "term_label": "chromatin"
}